{
  "term_label": "Unknown molecular function",
  "gene": "UniProtKB:Q96RK4",
  "gene_symbol": "BBS4",
  "gene_name": "Bardet-Biedl syndrome 4 protein",
  "term_id": "UNKNOWN:0001"
}